{
  "term_label": "RNA polymerase II cis-regulatory region sequence-specific DNA binding",
  "gene_name": "Zinc finger and BTB domain-containing protein 26",
  "gene": "UniProtKB:Q9HCK0",
  "term_id": "GO:0000978",
  "gene_symbol": "ZBTB26"
}